{
  "term_label": "regulation of filopodium assembly",
  "gene": "UniProtKB:P60953",
  "gene_symbol": "CDC42",
  "term_id": "GO:0051489",
  "gene_name": "Cell division control protein 42 homolog"
}